{
  "gene": "UniProtKB:Q8NHV1",
  "term_label": "GTPase activity",
  "term_id": "GO:0003924",
  "gene_symbol": "GIMAP7",
  "gene_name": "GTPase IMAP family member 7"
}